{
  "gene_symbol": "SHPK",
  "term_id": "GO:0009052",
  "gene_name": "Sedoheptulokinase",
  "gene": "UniProtKB:Q9UHJ6",
  "term_label": "pentose-phosphate shunt, non-oxidative branch"
}